{
  "gene_symbol": "FITM1",
  "term_id": "GO:0005789",
  "gene": "UniProtKB:A5D6W6",
  "gene_name": "Fat storage-inducing transmembrane protein 1",
  "term_label": "endoplasmic reticulum membrane"
}